carbon phosphorus lyase complex [GO:1904176] (cellular component) Relationships: is a type of catalytic complex [GO:1902494] Definition: A protein complex which is capable of carbon phosphorus lyase activity. Note: An example of this is PhnJ in E. coli (P16688) in PMID:22089136 (inferred from direct assay). References: PMID:17993513, PMID:21705661, PMID:22089136, PMID:23830682 Sources: GOC:TermGenie, GOC:bhm, GO_REF:0000088